{
  "term_label": "neutrophil chemotaxis",
  "gene_name": "C-C motif chemokine 28",
  "gene_symbol": "CCL28",
  "term_id": "GO:0030593",
  "gene": "UniProtKB:Q9NRJ3"
}